{
  "term_label": "Unknown cellular component",
  "term_id": "UNKNOWN:0003",
  "gene": "UniProtKB:A6NDA9",
  "gene_symbol": "LRIT2",
  "gene_name": "Leucine-rich repeat, immunoglobulin-like domain and transmembrane domain-containing protein 2"
}